{
  "term_label": "DNA-binding transcription factor activity, RNA polymerase II-specific",
  "gene_symbol": "DUX4L3",
  "gene": "UniProtKB:P0CJ86",
  "term_id": "GO:0000981",
  "gene_name": "Double homeobox protein 4-like protein 3"
}